{
  "term_label": "intracellular iron ion homeostasis",
  "term_id": "GO:0006879",
  "gene": "UniProtKB:P49281",
  "gene_symbol": "SLC11A2",
  "gene_name": "Natural resistance-associated macrophage protein 2"
}